{
  "term_id": "GO:0007286",
  "gene": "UniProtKB:Q9BXA6",
  "gene_name": "Testis-specific serine_threonine-protein kinase 6",
  "gene_symbol": "TSSK6",
  "term_label": "spermatid development"
}